{
  "gene_name": "Syntaxin-binding protein 2",
  "gene_symbol": "STXBP2",
  "term_label": "plasma membrane",
  "term_id": "GO:0005886",
  "gene": "UniProtKB:Q15833"
}